{
  "term_id": "UNKNOWN:0002",
  "gene_symbol": "RLBP1",
  "gene_name": "Retinaldehyde-binding protein 1",
  "term_label": "Unknown biological process",
  "gene": "UniProtKB:P12271"
}